positive regulation of cytokinesis [GO:0032467] (biological process) Subtypes: positive regulation of mitotic cytokinesis [GO:1903490], GO:2000076, positive regulation of FtsZ-dependent cytokinesis [GO:2000246], GO:2000433 Definition: Any process that activates or increases the frequency, rate or extent of the division of the cytoplasm of a cell, and its separation into two daughter cells. Relationships: is a type of regulation of cytokinesis [GO:0032465]; is a type of positive regulation of cell division [GO:0051781]; is a type of positive regulation of cell cycle process [GO:0090068]; positively regulates cytokinesis [GO:0000910] Also known as: up regulation of cytokinesis, up-regulation of cytokinesis, upregulation of cytokinesis, activation of cytokinesis, stimulation of cytokinesis, positive regulation of cell cycle cytokinesis Sources: GOC:mah